positive regulation of chromosome separation [GO:1905820] (biological process) Relationships: is a type of positive regulation of cell cycle process [GO:0090068]; is a type of regulation of chromosome separation [GO:1905818]; positively regulates chromosome separation [GO:0051304] References: PMID:21795393 Sources: GOC:TermGenie, GOC:bhm, GO_REF:0000058 Subtypes: positive regulation of mitotic sister chromatid separation [GO:1901970], positive regulation of meiotic chromosome separation [GO:1905134] Also known as: up regulation of chromosome separation, up-regulation of chromosome separation, upregulation of chromosome separation, activation of chromosome separation, activation of rDNA separation, positive regulation of rDNA separation, up regulation of rDNA separation, up-regulation of rDNA separation, upregulation of rDNA separation, activation of chromatid release, positive regulation of chromatid release, up regulation of chromatid release, up-regulation of chromatid release, upregulation of chromatid release Definition: Any process that activates or increases the frequency, rate or extent of chromosome separation.